collagen type XI trimer [GO:0005592] (cellular component) Relationships: is a type of fibrillar collagen trimer [GO:0005583] References: PMID:7642541 Definition: A collagen heterotrimer containing type XI and type II alpha chains in alpha1(XI) alpha2(XI) alpha1(II) trimers; type XI collagen triple helices associate to form fibrils.